imaginal disc-derived male genitalia development [GO:0007485] (biological process) Also known as: male genital development Relationships: is a type of imaginal disc-derived genitalia development [GO:0007484] Definition: The process whose specific outcome is the progression of the male genitalia over time, from formation as part of the genital disc to the mature structure. An example of this is found in Drosophila melanogaster. Sources: GOC:ai, GOC:sensu